{
  "gene_symbol": "PPIL3",
  "term_label": "peptidyl-prolyl cis-trans isomerase activity",
  "gene_name": "Peptidyl-prolyl cis-trans isomerase-like 3",
  "gene": "UniProtKB:Q9H2H8",
  "term_id": "GO:0003755"
}